negative regulation of epithelial cell proliferation involved in lung morphogenesis [GO:2000795] (biological process) Relationships: is a type of negative regulation of epithelial cell proliferation [GO:0050680]; is a type of regulation of epithelial cell proliferation involved in lung morphogenesis [GO:2000794]; RO_0002212 epithelial cell proliferation involved in lung morphogenesis [GO:0060502] References: PMID:21513708 Definition: Any process that stops, prevents or reduces the frequency, rate or extent of epithelial cell proliferation involved in lung morphogenesis.